{
  "gene_symbol": "HBD",
  "gene": "UniProtKB:P02042",
  "term_label": "haptoglobin-hemoglobin complex",
  "gene_name": "Hemoglobin subunit delta",
  "term_id": "GO:0031838"
}